trehalose O-mycolyltransferase activity [GO:0050348] (molecular function) Relationships: is a type of acyltransferase activity, transferring groups other than amino-acyl groups [GO:0016747] Sources: EC:2.3.1.122, RHEA:23472 Definition: Catalysis of the reaction: 2 alpha,alpha'-trehalose 6-mycolate = alpha,alpha'-trehalose 6,6'-bismycolate + alpha,alpha-trehalose. Also known as: alpha,alpha'-trehalose 6-monomycolate:alpha,alpha'-trehalose mycolyltransferase activity, alpha,alpha'-trehalose-6-mycolate:alpha,alpha'-trehalose-6-mycolate 6'-mycolyltransferase activity